{
  "term_id": "UNKNOWN:0002",
  "gene_symbol": "LRRCC1",
  "gene": "UniProtKB:Q9C099",
  "gene_name": "Leucine-rich repeat and coiled-coil domain-containing protein 1",
  "term_label": "Unknown biological process"
}